{
  "gene_symbol": "IGHV4-30-2",
  "term_id": "UNKNOWN:0003",
  "term_label": "Unknown cellular component",
  "gene": "UniProtKB:A0A087WSY4",
  "gene_name": "Immunoglobulin heavy variable 4-30-2"
}